{
  "gene_symbol": "LIPF",
  "term_label": "Unknown cellular component",
  "term_id": "UNKNOWN:0003",
  "gene": "UniProtKB:P07098",
  "gene_name": "Gastric triacylglycerol lipase"
}